{
  "gene_symbol": "NLRP1",
  "term_label": "nucleus",
  "gene_name": "NACHT, LRR and PYD domains-containing protein 1",
  "gene": "UniProtKB:Q9C000",
  "term_id": "GO:0005634"
}